{
  "term_id": "GO:0048704",
  "gene": "UniProtKB:P31249",
  "gene_name": "Homeobox protein Hox-D3",
  "term_label": "embryonic skeletal system morphogenesis",
  "gene_symbol": "HOXD3"
}